complement component C1 complex [GO:0005602] (cellular component) Also known as: complement component C1q complex Relationships: is a type of protein-containing complex [GO:0032991]; BFO_0000050 extracellular region [GO:0005576]; has part GO:0062167 Sources: GOC:add, ISBN:0781735149 Definition: A protein complex composed of six subunits of C1q, each formed of the three homologous polypeptide chains C1QA, C1QB, and C1QB, and tetramer of two C1QR and two C1QS polypeptide chains.